{
  "gene": "UniProtKB:Q8N7Z2",
  "term_id": "UNKNOWN:0001",
  "term_label": "Unknown molecular function",
  "gene_name": "Golgin subfamily A member 6-like protein 1",
  "gene_symbol": "GOLGA6L1"
}